{
  "term_id": "GO:0016757",
  "term_label": "glycosyltransferase activity",
  "gene_name": "Exostosin-2",
  "gene_symbol": "EXT2",
  "gene": "UniProtKB:Q93063"
}